{
  "gene_symbol": "LTA",
  "term_label": "cytokine activity",
  "term_id": "GO:0005125",
  "gene_name": "Lymphotoxin-alpha",
  "gene": "UniProtKB:P01374"
}